regulation of single-strand break repair via homologous recombination [GO:1903110] (biological process) Subtypes: GO:1903111, positive regulation of single-strand break repair via homologous recombination [GO:1903112] Definition: Any process that modulates the frequency, rate or extent of single-strand break repair via homologous recombination. References: PMID:24339919 Sources: GOC:TermGenie, GOC:bhm, GO_REF:0000058 Relationships: is a type of GO:0000018; is_a GO:1903516; regulates single-strand break repair via homologous recombination [GO:1990396]